cerebellar Purkinje cell layer development [GO:0021680] (biological process) Definition: The process whose specific outcome is the progression of the cerebellar Purkinje cell layer over time, from its formation to the mature structure. The Purkinje cell layer lies just underneath the molecular layer of the cerebellar cortex. It contains the neuronal cell bodies of the Purkinje cells that are arranged side by side in a single layer. Candelabrum interneurons are vertically oriented between the Purkinje cells. Purkinje neurons are inhibitory and provide the output of the cerebellar cortex through axons that project into the white matter. Extensive dendritic trees from the Purkinje cells extend upward in a single plane into the molecular layer where they synapse with parallel fibers of granule cells. Sources: GOC:cls, GOC:dgh, GOC:dph, GOC:jid, GO_REF:0000021 Relationships: is a type of GO:0048856; is part of GO:0021695